detection of pH by aortic body chemoreceptor signaling [GO:0003036] (biological process) Definition: The process in which information about the levels of hydrogen ions are received and are converted to a molecular signal by chemoreceptors in an aortic body. Relationships: is_a detection of pH by chemoreceptor signaling [GO:0003022]; is part of GO:0003033 Also known as: detection of pH by aortic body chemoreceptor signalling Sources: GOC:mtg_cardio